positive regulation of neuroepithelial cell differentiation [GO:1902913] (biological process) Definition: Any process that activates or increases the frequency, rate or extent of neuroepithelial cell differentiation. References: PMID:16916506 Sources: GOC:TermGenie, GOC:mr, GO_REF:0000058 Subtypes: positive regulation of odontoblast differentiation [GO:1901331] Also known as: up regulation of neuroepithelial cell differentiation, up-regulation of neuroepithelial cell differentiation, upregulation of neuroepithelial cell differentiation, activation of neuroepithelial cell differentiation Relationships: is a type of positive regulation of epithelial cell differentiation [GO:0030858]; positively regulates GO:0060563